{
  "gene": "UniProtKB:Q86U28",
  "gene_symbol": "ISCA2",
  "term_id": "GO:0051537",
  "term_label": "2 iron, 2 sulfur cluster binding",
  "gene_name": "Iron-sulfur cluster assembly 2 homolog, mitochondrial"
}